{
  "term_id": "GO:1990837",
  "gene_name": "Short stature homeobox protein 2",
  "gene": "UniProtKB:O60902",
  "gene_symbol": "SHOX2",
  "term_label": "sequence-specific double-stranded DNA binding"
}